{
  "gene_symbol": "AURKA",
  "gene": "UniProtKB:O14965",
  "term_label": "mitotic spindle organization",
  "term_id": "GO:0007052",
  "gene_name": "Aurora kinase A"
}